{
  "gene_name": "Rho-related GTP-binding protein RhoU",
  "gene": "UniProtKB:Q7L0Q8",
  "term_id": "GO:0003924",
  "term_label": "GTPase activity",
  "gene_symbol": "RHOU"
}